{
  "gene_name": "Nuclear exosome regulator NRDE2",
  "gene": "UniProtKB:Q9H7Z3",
  "term_label": "Unknown molecular function",
  "gene_symbol": "NRDE2",
  "term_id": "UNKNOWN:0001"
}